{
  "gene": "UniProtKB:P17405",
  "gene_symbol": "SMPD1",
  "term_id": "GO:0006685",
  "term_label": "sphingomyelin catabolic process",
  "gene_name": "Sphingomyelin phosphodiesterase"
}